{
  "gene": "UniProtKB:Q8TF66",
  "term_id": "GO:0005886",
  "gene_name": "Leucine-rich repeat-containing protein 15",
  "gene_symbol": "LRRC15",
  "term_label": "plasma membrane"
}